pyrimidine nucleotide metabolic process [GO:0006220] (biological process) Definition: The chemical reactions and pathways involving a pyrimidine nucleotide, a compound consisting of nucleoside (a pyrimidine base linked to a deoxyribose or ribose sugar) esterified with a phosphate group at either the 3' or 5'-hydroxyl group of the sugar. Relationships: is a type of GO:0009117; is a type of pyrimidine-containing compound metabolic process [GO:0072527] Also known as: pyrimidine metabolic process, pyrimidine metabolism, pyrimidine nucleotide metabolism Sources: GOC:go_curators, ISBN:0198506732 Subtypes: pyrimidine nucleotide biosynthetic process [GO:0006221], pyrimidine nucleotide catabolic process [GO:0006244], GO:0009218, pyrimidine deoxyribonucleotide metabolic process [GO:0009219], pyrimidine nucleotide interconversion [GO:0015953]